protein deubiquitination [GO:0016579] (biological process) Relationships: is a type of GO:0070646; has part cysteine-type deubiquitinase activity [GO:0004843] Definition: The removal of one or more ubiquitin groups from a protein. Regulation: RO_0002211 by GO:0090085; negatively regulated by negative regulation of protein deubiquitination [GO:0090086]; positively regulated by positive regulation of protein deubiquitination [GO:1903003] Subtypes: monoubiquitinated protein deubiquitination [GO:0035520], GO:0035523, protein K11-linked deubiquitination [GO:0035871], protein K6-linked deubiquitination [GO:0044313], protein K63-linked deubiquitination [GO:0070536], protein K48-linked deubiquitination [GO:0071108], GO:0071947, GO:1990108, GO:1990167, protein K33-linked deubiquitination [GO:1990168] Sources: GOC:ai Also known as: deubiquitination, protein deubiquitinylation, protein deubiquitylation